corneal epithelial cell migration [GO:0061581] (biological process) Relationships: is a type of epithelial cell migration [GO:0010631] Sources: GOC:dph Definition: The orderly movement of a corneal epithelial cell from one site to another, often during the development of a multicellular organism.